detection of mechanical stimulus involved in sensory perception of gravity [GO:0070999] (biological process) Sources: GOC:dos, GOC:mah Relationships: is a type of GO:0009590; is a type of detection of mechanical stimulus involved in sensory perception [GO:0050974]; is part of sensory perception of gravity [GO:0070998] Definition: The series of events involved in the perception of gravity in which a sensory mechanical stimulus is received and converted into a molecular signal.